{
  "gene_name": "Collagen alpha-1(IX) chain",
  "gene": "UniProtKB:P20849",
  "term_id": "GO:0031012",
  "gene_symbol": "COL9A1",
  "term_label": "extracellular matrix"
}